effector-mediated suppression of host innate immune response [GO:0140403] (biological process) Definition: A process mediated by a molecule secreted by a symbiont that results in the suppression of a host innate immune response. The host is defined as the larger of the organisms involved in a symbiotic interaction. References: PMID:21467214, PMID:30584105 Also known as: effector dependent suppression of host immune innate response by symbiont, effector triggered suppression of host immune innate response by symbiont, effector-dependent suppression of host immune innate response by symbiont, effector-mediated suppression of host immune innate response by symbiont, effector-mediated suppression of host innate immune response by symbiont, effector-mediated suppression of host innate immunity, effector-triggered suppression of host immune innate response by symbiont Relationships: is a type of symbiont-mediated suppression of host innate immune response [GO:0052170]; is a type of effector-mediated perturbation of host innate immune response by symbiont [GO:0140404]; is a type of effector-mediated suppression of host defense response [GO:0140590] Subtypes: GO:0034055, effector-mediated suppression of host pattern-triggered immunity [GO:0052034]